{
  "gene_symbol": "A0A2R8Y556",
  "gene": "UniProtKB:A0A2R8Y556",
  "term_id": "UNKNOWN:0002",
  "term_label": "Unknown biological process",
  "gene_name": "Uncharacterized protein"
}